{
  "term_id": "GO:0016064",
  "gene_symbol": "IGHV3-38-3",
  "gene_name": "Probable non-functional immunoglobulin heavy variable 3-38-3",
  "term_label": "immunoglobulin mediated immune response",
  "gene": "UniProtKB:P0DTE1"
}